{
  "gene_name": "Cytochrome P450 2C9",
  "gene": "UniProtKB:P11712",
  "term_id": "GO:0005737",
  "gene_symbol": "CYP2C9",
  "term_label": "cytoplasm"
}